cinnamate beta-D-glucosyltransferase activity [GO:0050412] (molecular function) Definition: Catalysis of the reaction: trans-cinnamate + UDP-D-glucose = 1-O-trans-cinnamoyl-beta-D-glucopyranose + UDP. Sources: EC:2.4.1.177, RHEA:13437 Relationships: is a type of UDP-glucosyltransferase activity [GO:0035251] Also known as: cinnamate b-D-glucosyltransferase activity, cinnamate glucosyltransferase activity, UDP-glucose:trans-cinnamate beta-D-glucosyltransferase activity, UDPG:t-cinnamate glucosyltransferase activity, UDPglucose:trans-cinnamate beta-D-glucosyltransferase activity, uridine diphosphoglucose-cinnamate glucosyltransferase activity